{
  "term_id": "UNKNOWN:0002",
  "gene_name": "Putative uncharacterized protein CDRT15P3",
  "gene_symbol": "CDRT15P3",
  "gene": "UniProtKB:P0DPF6",
  "term_label": "Unknown biological process"
}